{
  "gene_symbol": "LTK",
  "gene_name": "Leukocyte tyrosine kinase receptor",
  "gene": "UniProtKB:P29376",
  "term_id": "GO:0005886",
  "term_label": "plasma membrane"
}